{
  "term_id": "UNKNOWN:0002",
  "gene_symbol": "MCFD2",
  "gene": "UniProtKB:Q8NI22",
  "term_label": "Unknown biological process",
  "gene_name": "Multiple coagulation factor deficiency protein 2"
}